diadenosine polyphosphate biosynthetic process [GO:0015960] (biological process) Subtypes: diadenosine triphosphate biosynthetic process [GO:0015963], diadenosine tetraphosphate biosynthetic process [GO:0015966] Sources: GOC:ai Definition: The chemical reactions and pathways resulting in the formation of diadenosine polyphosphate, a derivative of the nucleoside adenosine with phosphate groups attached. Also known as: diadenosine polyphosphate anabolism, diadenosine polyphosphate biosynthesis, diadenosine polyphosphate formation, diadenosine polyphosphate synthesis Relationships: is_a nucleotide biosynthetic process [GO:0009165]; is a type of diadenosine polyphosphate metabolic process [GO:0015959]